{
  "term_label": "small-subunit processome",
  "gene": "UniProtKB:Q8NEJ9",
  "gene_name": "Neuroguidin",
  "term_id": "GO:0032040",
  "gene_symbol": "NGDN"
}